{
  "term_id": "UNKNOWN:0002",
  "term_label": "Unknown biological process",
  "gene": "UniProtKB:P42025",
  "gene_name": "Beta-centractin",
  "gene_symbol": "ACTR1B"
}